{
  "gene": "UniProtKB:Q8IVB4",
  "gene_symbol": "SLC9A9",
  "term_label": "potassium ion transmembrane transport",
  "gene_name": "Sodium_hydrogen exchanger 9",
  "term_id": "GO:0071805"
}